{
  "gene": "UniProtKB:Q99747",
  "term_label": "intracellular protein transport",
  "gene_symbol": "NAPG",
  "gene_name": "Gamma-soluble NSF attachment protein",
  "term_id": "GO:0006886"
}